{
  "gene_symbol": "OSBPL6",
  "gene_name": "Oxysterol-binding protein-related protein 6",
  "term_label": "Unknown biological process",
  "term_id": "UNKNOWN:0002",
  "gene": "UniProtKB:Q9BZF3"
}